{
  "term_label": "spindle pole",
  "gene_symbol": "AUNIP",
  "gene": "UniProtKB:Q9H7T9",
  "gene_name": "Aurora kinase A and ninein-interacting protein",
  "term_id": "GO:0000922"
}